hydrolase activity, acting on glycosyl bonds [GO:0016798] (molecular function) Subtypes: GO:0004553, hydrolase activity, hydrolyzing N-glycosyl compounds [GO:0016799], sulfoquinovosidase activity [GO:1990929] Sources: GOC:jl Relationships: is a type of GO:0016787 Also known as: glycosidase activity, N-glycosylase, glycosylase Definition: Catalysis of the hydrolysis of any glycosyl bond.